head development [GO:0060322] (biological process) Sources: GOC:dph Definition: The biological process whose specific outcome is the progression of a head from an initial condition to its mature state. The head is the anterior-most division of the body. Subtypes: anterior head development [GO:0097065] Relationships: is a type of anatomical structure development [GO:0048856]